{
  "gene_symbol": "IREB2",
  "gene": "UniProtKB:P48200",
  "gene_name": "Iron-responsive element-binding protein 2",
  "term_label": "4 iron, 4 sulfur cluster binding",
  "term_id": "GO:0051539"
}